{
  "gene": "UniProtKB:P13945",
  "term_id": "GO:0043410",
  "gene_symbol": "ADRB3",
  "gene_name": "Beta-3 adrenergic receptor",
  "term_label": "positive regulation of MAPK cascade"
}